{
  "gene_name": "Putative uncharacterized protein PRO1933",
  "gene_symbol": "PRO1933",
  "term_id": "UNKNOWN:0001",
  "gene": "UniProtKB:Q9H354",
  "term_label": "Unknown molecular function"
}